{
  "term_label": "polynucleotide 5'-phosphatase activity",
  "gene_name": "RNA_RNP complex-1-interacting phosphatase",
  "gene_symbol": "DUSP11",
  "gene": "UniProtKB:O75319",
  "term_id": "GO:0004651"
}